{
  "term_label": "Unknown cellular component",
  "gene_symbol": "MISP",
  "term_id": "UNKNOWN:0003",
  "gene": "UniProtKB:Q8IVT2",
  "gene_name": "Mitotic interactor and substrate of PLK1"
}